D-ribose 5-phosphate catabolic process [GO:1901279] (biological process) Definition: The chemical reactions and pathways resulting in the breakdown of D-ribose 5-phosphate. Also known as: D-ribose 5-phosphate breakdown, D-ribose 5-phosphate catabolism, D-ribose 5-phosphate degradation Relationships: is a type of GO:0019693; is a type of GO:0046434; is a type of carbohydrate derivative catabolic process [GO:1901136] Sources: GOC:TermGenie, GOC:yaf, UniPathway:UPA00293